negative regulation of MHC class I biosynthetic process [GO:0045344] (biological process) Definition: Any process that stops, prevents, or reduces the frequency, rate or extent of the chemical reactions and pathways resulting in the formation of MHC class I. Sources: GOC:go_curators Also known as: down regulation of MHC class I biosynthetic process, down-regulation of MHC class I biosynthetic process, downregulation of MHC class I biosynthetic process, negative regulation of MHC class I anabolism, negative regulation of MHC class I biosynthesis, negative regulation of MHC class I formation, negative regulation of MHC class I synthesis, negative regulation of major histocompatibility complex class I biosynthesis, negative regulation of major histocompatibility complex class I biosynthetic process, inhibition of MHC class I biosynthetic process Relationships: is a type of negative regulation of macromolecule biosynthetic process [GO:0010558]; is a type of regulation of MHC class I biosynthetic process [GO:0045343]; negatively regulates MHC class I biosynthetic process [GO:0045341]